{
  "gene_symbol": "MCHR1",
  "term_label": "neuropeptide binding",
  "gene": "UniProtKB:Q99705",
  "term_id": "GO:0042923",
  "gene_name": "Melanin-concentrating hormone receptor 1"
}